positive regulation of complement activation, classical pathway [GO:0045960] (biological process) Definition: Any process that activates or increases the frequency, rate or extent of complement activation by the classical pathway. Sources: GOC:go_curators Also known as: positive regulation of complement cascade, classical pathway, up regulation of complement activation, classical pathway, up-regulation of complement activation, classical pathway, upregulation of complement activation, classical pathway, activation of complement activation, classical pathway, stimulation of complement activation, classical pathway Relationships: is a type of positive regulation of humoral immune response mediated by circulating immunoglobulin [GO:0002925]; is a type of regulation of complement activation, classical pathway [GO:0030450]; is_a positive regulation of complement activation [GO:0045917]; positively regulates GO:0006958